{
  "gene_name": "HLA class I histocompatibility antigen, B alpha chain",
  "term_label": "external side of plasma membrane",
  "gene_symbol": "HLA-B",
  "term_id": "GO:0009897",
  "gene": "UniProtKB:P01889"
}